cell adhesion involved in single-species biofilm formation in or on host organism [GO:0043707] (BP) Relationships: is a type of cell adhesion involved in single-species biofilm formation [GO:0043709]; is part of single-species biofilm formation in or on host organism [GO:0044407] Also known as: cell adhesion during single-species biofilm formation in or on host organism Definition: The attachment of a cell to either a host cell or a microbial cell of the same species, or to an underlying host substrate, such as the extracellular matrix, via cell adhesion molecules, occurring during the formation of a biofilm in or on a host species. Sources: GOC:jl